{
  "gene": "UniProtKB:A4D2H0",
  "term_id": "GO:0009306",
  "term_label": "protein secretion",
  "gene_name": "cTAGE family member 15",
  "gene_symbol": "CTAGE15"
}